{
  "gene_name": "Nucleolar protein 8",
  "gene": "UniProtKB:Q76FK4",
  "term_id": "GO:1902570",
  "term_label": "protein localization to nucleolus",
  "gene_symbol": "NOL8"
}